{
  "gene_symbol": "GPR32",
  "gene": "UniProtKB:O75388",
  "gene_name": "Probable G-protein coupled receptor 32",
  "term_label": "complement receptor mediated signaling pathway",
  "term_id": "GO:0002430"
}